{
  "gene_name": "Two pore channel protein 2",
  "gene": "UniProtKB:Q8NHX9",
  "gene_symbol": "TPCN2",
  "term_label": "lysosomal membrane",
  "term_id": "GO:0005765"
}